iron chelate transmembrane transporter activity [GO:0015603] (molecular function) Definition: Enables the transfer of an iron chelate from one side of a membrane to the other. An iron chelate is a heterocyclic compound having a metal ion attached by coordinate bonds to at least two nonmetal ions. Relationships: is a type of GO:0022857; is part of GO:0033214 References: PMID:17660286 Subtypes: siderophore-iron transmembrane transporter activity [GO:0015343], ferric enterobactin:proton symporter activity [GO:0015345], ABC-type ferric-enterobactin transporter activity [GO:0015624], GO:0015625, GO:0019535, iron-nicotianamine transmembrane transporter activity [GO:0051980]